aspartate dehydrogenase [NAD(P)+] activity [GO:0033735] (molecular function) Also known as: aspartate dehydrogenase NAD activity, aspartate dehydrogenase NADP activity, L-aspartate:NAD(P)+ oxidoreductase (deaminating) activity, NAD-dependent aspartate dehydrogenase activity, NADH2-dependent aspartate dehydrogenase activity, NADP+-dependent aspartate dehydrogenase activity Relationships: is a type of oxidoreductase activity, acting on the CH-NH2 group of donors [GO:0016638] Sources: EC:1.4.1.21 Definition: Catalysis of the reaction: L-aspartate + H2O + NAD(P)+ = oxaloacetate + NH3 + NAD(P)H + H+.